regulation of killing of cells of another organism [GO:0051709] (biological process) Subtypes: negative regulation of killing of cells of another organism [GO:0051711], GO:0051712, symbiont-mediated perturbation of host apoptosis [GO:0052150], regulation of neutrophil mediated killing of symbiont cell [GO:0070949] Sources: GOC:ai Relationships: is a type of GO:0031341; is a type of modulation of process of another organism [GO:0035821]; regulates GO:0031640 Definition: Any process that modulates the frequency, rate or extent of the killing by an organism of cells in another organism. Also known as: regulation of killing of cells of other organism, modulation by organism of apoptotic process in other organism involved in symbiotic interaction, modulation of programmed cell death in other organism, modulation of programmed cell death in other organism involved in symbiotic interaction